{
  "gene_name": "Scavenger receptor cysteine-rich type 1 protein M160",
  "term_label": "external side of plasma membrane",
  "term_id": "GO:0009897",
  "gene": "UniProtKB:Q9NR16",
  "gene_symbol": "CD163L1"
}